{
  "gene_name": "Junctional adhesion molecule-like",
  "term_id": "GO:0050839",
  "gene": "UniProtKB:Q86YT9",
  "term_label": "cell adhesion molecule binding",
  "gene_symbol": "JAML"
}